isoquinoline 1-oxidoreductase activity [GO:0047121] (molecular function) Relationships: is a type of oxidoreductase activity, acting on the CH-CH group of donors [GO:0016627] Sources: EC:1.3.99.16, RHEA:11588 Also known as: isoquinoline:acceptor 1-oxidoreductase (hydroxylating) Definition: Catalysis of the reaction: A + H2O + isoquinoline = AH(2) + isoquinolin-1(2H)-one.